{
  "gene_symbol": "COL4A1",
  "gene_name": "Collagen alpha-1(IV) chain",
  "term_label": "extracellular matrix",
  "term_id": "GO:0031012",
  "gene": "UniProtKB:P02462"
}